regulation of hematopoietic stem cell proliferation [GO:1902033] (biological process) Subtypes: GO:1902034, positive regulation of hematopoietic stem cell proliferation [GO:1902035] Relationships: is a type of regulation of stem cell proliferation [GO:0072091]; regulates hematopoietic stem cell proliferation [GO:0071425] Also known as: regulation of hemopoietic stem cell proliferation Definition: Any process that modulates the frequency, rate or extent of hematopoietic stem cell proliferation. References: PMID:23403623 Sources: GOC:TermGenie